response to arsenic-containing substance [GO:0046685] (biological process) Also known as: response to arsenic, arsenate sensitivity/resistance Sources: GOC:hjd, ISBN:0721662544 Subtypes: cellular response to arsenic-containing substance [GO:0071243], response to arsenite(3-) [GO:1903840], response to arsenite ion [GO:1903842], response to sodium arsenite [GO:1903935] Relationships: is a type of response to chemical [GO:0042221] Definition: Any process that results in a change in state or activity of a cell or an organism (in terms of movement, secretion, enzyme production, gene expression, etc.) as a result of an arsenic stimulus from compounds containing arsenic, including arsenates, arsenites, and arsenides.